{
  "gene_symbol": "PIGN",
  "gene": "UniProtKB:O95427",
  "gene_name": "GPI ethanolamine phosphate transferase 1",
  "term_label": "mannose-ethanolamine phosphotransferase activity",
  "term_id": "GO:0051377"
}